{
  "gene": "UniProtKB:Q86YV9",
  "term_id": "GO:0031084",
  "gene_symbol": "HPS6",
  "gene_name": "BLOC-2 complex member HPS6",
  "term_label": "BLOC-2 complex"
}